{
  "gene_name": "Lipopolysaccharide-induced tumor necrosis factor-alpha factor",
  "term_label": "regulation of cytokine production",
  "gene_symbol": "LITAF",
  "gene": "UniProtKB:Q99732",
  "term_id": "GO:0001817"
}